{
  "term_label": "neural crest cell migration",
  "gene_symbol": "SEMA3G",
  "gene": "UniProtKB:Q9NS98",
  "gene_name": "Semaphorin-3G",
  "term_id": "GO:0001755"
}